intracellular ornithine homeostasis [GO:0090462] (biological process) Definition: A homeostatic process involved in the maintenance of a steady state level of orthinine within a cell. Sources: GOC:tb Also known as: cellular ornithine homeostasis, ornithine homeostasis Relationships: is a type of GO:0080144